{
  "term_id": "GO:0000978",
  "gene_symbol": "NR2E1",
  "gene_name": "Nuclear receptor subfamily 2 group E member 1",
  "gene": "UniProtKB:Q9Y466",
  "term_label": "RNA polymerase II cis-regulatory region sequence-specific DNA binding"
}